{
  "gene_name": "Alkaline ceramidase 2",
  "gene_symbol": "ACER2",
  "term_id": "GO:0000139",
  "gene": "UniProtKB:Q5QJU3",
  "term_label": "Golgi membrane"
}